regulation of glial cell apoptotic process [GO:0034350] (biological process) Also known as: regulation of glial cell apoptosis Relationships: is a type of regulation of apoptotic process [GO:0042981]; regulates glial cell apoptotic process [GO:0034349] Subtypes: negative regulation of glial cell apoptotic process [GO:0034351], GO:0034352, regulation of oligodendrocyte apoptotic process [GO:1900141] Definition: Any process that modulates the frequency, rate, or extent of glial cell apoptotic process. Sources: GOC:mah, GOC:mtg_apoptosis